{
  "gene_symbol": "MYL12A",
  "gene": "UniProtKB:P19105",
  "term_id": "GO:0032036",
  "term_label": "myosin heavy chain binding",
  "gene_name": "Myosin regulatory light chain 12A"
}